{
  "term_id": "UNKNOWN:0001",
  "gene": "UniProtKB:P13671",
  "gene_name": "Complement component C6",
  "gene_symbol": "C6",
  "term_label": "Unknown molecular function"
}